{
  "term_label": "Golgi organization",
  "term_id": "GO:0007030",
  "gene_symbol": "COG7",
  "gene_name": "Conserved oligomeric Golgi complex subunit 7",
  "gene": "UniProtKB:P83436"
}